{
  "gene": "UniProtKB:Q9NRC6",
  "term_label": "cell projection",
  "gene_name": "Spectrin beta chain, non-erythrocytic 5",
  "term_id": "GO:0042995",
  "gene_symbol": "SPTBN5"
}